{
  "gene_name": "SH2 domain-containing adapter protein F",
  "gene_symbol": "SHF",
  "term_id": "UNKNOWN:0002",
  "term_label": "Unknown biological process",
  "gene": "UniProtKB:Q7M4L6"
}